{
  "gene_name": "Putative uncharacterized protein LOC400499",
  "term_label": "Unknown cellular component",
  "gene_symbol": "Q6ZTK2",
  "term_id": "UNKNOWN:0003",
  "gene": "UniProtKB:Q6ZTK2"
}